{
  "term_id": "GO:0000813",
  "gene_name": "Vacuolar protein sorting-associated protein 37A",
  "term_label": "ESCRT I complex",
  "gene": "UniProtKB:Q8NEZ2",
  "gene_symbol": "VPS37A"
}